{
  "gene_name": "Inhibitor of nuclear factor kappa-B kinase-interacting protein",
  "term_label": "Unknown molecular function",
  "term_id": "UNKNOWN:0001",
  "gene_symbol": "IKBIP",
  "gene": "UniProtKB:Q70UQ0"
}